{
  "term_label": "leukocyte cell-cell adhesion",
  "gene_name": "CD177 antigen",
  "gene": "UniProtKB:Q8N6Q3",
  "term_id": "GO:0007159",
  "gene_symbol": "CD177"
}